{
  "term_label": "negative regulation of hippo signaling",
  "gene_name": "Wilms tumor protein 1-interacting protein",
  "term_id": "GO:0035331",
  "gene_symbol": "WTIP",
  "gene": "UniProtKB:A6NIX2"
}